{
  "gene_symbol": "CDY2A",
  "term_id": "GO:0061628",
  "gene": "UniProtKB:Q9Y6F7",
  "term_label": "histone H3K27me3 reader activity",
  "gene_name": "Testis-specific chromodomain protein Y 2"
}